{
  "gene": "UniProtKB:Q14807",
  "term_label": "microtubule binding",
  "gene_name": "Kinesin-like protein KIF22",
  "term_id": "GO:0008017",
  "gene_symbol": "KIF22"
}